{
  "gene_name": "Golgin subfamily A member 8R",
  "gene_symbol": "GOLGA8R",
  "term_label": "Golgi cis cisterna",
  "gene": "UniProtKB:I6L899",
  "term_id": "GO:0000137"
}